central B cell positive selection [GO:0002348] (biological process) Sources: GOC:jal Relationships: is a type of GO:0002340; is a type of B cell positive selection [GO:0002346] Also known as: central B lymphocyte positive selection, central B-cell positive selection, central B-lymphocyte positive selection Definition: Any process leading to positive selection of B cells in the bone marrow. Positive selection is the process in which B or T cells are selected to survive based on signaling through their antigen receptors.